{
  "term_id": "GO:0010468",
  "gene_symbol": "TRIM4",
  "gene_name": "E3 ubiquitin-protein ligase TRIM4",
  "term_label": "regulation of gene expression",
  "gene": "UniProtKB:Q9C037"
}